{
  "gene": "UniProtKB:Q9NP72",
  "gene_name": "Ras-related protein Rab-18",
  "gene_symbol": "RAB18",
  "term_label": "Golgi apparatus",
  "term_id": "GO:0005794"
}